{
  "gene": "UniProtKB:Q96MM7",
  "gene_symbol": "HS6ST2",
  "term_id": "GO:0015012",
  "gene_name": "Heparan-sulfate 6-O-sulfotransferase 2",
  "term_label": "heparan sulfate proteoglycan biosynthetic process"
}